{
  "gene": "UniProtKB:P04196",
  "gene_name": "Histidine-rich glycoprotein",
  "gene_symbol": "HRG",
  "term_id": "GO:0061844",
  "term_label": "antimicrobial humoral immune response mediated by antimicrobial peptide"
}